{
  "gene_symbol": "E2F5",
  "gene": "UniProtKB:Q15329",
  "term_id": "GO:0006357",
  "term_label": "regulation of transcription by RNA polymerase II",
  "gene_name": "Transcription factor E2F5"
}